sno(s)RNA metabolic process [GO:0016074] (biological process) Subtypes: sno(s)RNA transcription [GO:0009302], sno(s)RNA catabolic process [GO:0016077], box C/D sno(s)RNA metabolic process [GO:0033967], box H/ACA sno(s)RNA metabolic process [GO:0033979], sno(s)RNA processing [GO:0043144] Relationships: is a type of RNA metabolic process [GO:0016070] Sources: GOC:krc Regulation: regulated by regulation of snoRNA metabolic process [GO:1903323]; negatively regulated by GO:1903324; positively regulated by positive regulation of snoRNA metabolic process [GO:1903325] Also known as: box C/D sRNA metabolic process, snoRNA metabolism Definition: The chemical reactions and pathways involving snoRNA, small nucleolar RNA, any of a class of small RNAs that are associated with the eukaryotic nucleus as components of small nucleolar ribonucleoproteins. They participate in the processing or modifications of many RNAs, mostly ribosomal RNAs (rRNAs) though snoRNAs are also known to target other classes of RNA, including spliceosomal RNAs, tRNAs, and mRNAs via a stretch of sequence that is complementary to a sequence in the targeted RNA.